{
  "term_label": "cell surface",
  "term_id": "GO:0009986",
  "gene_name": "Fms-related tyrosine kinase 3 ligand",
  "gene": "UniProtKB:P49771",
  "gene_symbol": "FLT3LG"
}